diiodophenylpyruvate reductase (NAD+) activity [GO:0047860] (molecular function) Definition: Catalysis of the reaction: 3-(3,5-diiodo-4-hydroxyphenyl)lactate + NAD+ = 3-(3,5-diiodo-4-hydroxyphenyl)pyruvate + H+ + NADH. Relationships: is_a oxidoreductase activity, acting on the CH-OH group of donors, NAD or NADP as acceptor [GO:0016616] Sources: RHEA:20293 Also known as: 2-oxo acid reductase activity, 3-(3,5-diiodo-4-hydroxyphenyl)lactate:NAD+ oxidoreductase activity, KAR, aromatic alpha-keto acid